{
  "gene": "UniProtKB:P00748",
  "term_id": "GO:0007596",
  "term_label": "blood coagulation",
  "gene_symbol": "F12",
  "gene_name": "Coagulation factor XII"
}